{
  "gene_name": "Probable proton-coupled zinc antiporter SLC30A3",
  "gene_symbol": "SLC30A3",
  "term_id": "GO:0005385",
  "gene": "UniProtKB:Q99726",
  "term_label": "zinc ion transmembrane transporter activity"
}